{
  "gene_symbol": "TFAP4",
  "term_id": "GO:0006357",
  "gene": "UniProtKB:Q01664",
  "term_label": "regulation of transcription by RNA polymerase II",
  "gene_name": "Transcription factor AP-4"
}